{
  "gene": "UniProtKB:Q9UM63",
  "gene_name": "Zinc finger protein PLAGL1",
  "gene_symbol": "PLAGL1",
  "term_label": "regulation of immune system process",
  "term_id": "GO:0002682"
}